{
  "term_id": "GO:0007165",
  "gene_name": "Calcium_calmodulin-dependent protein kinase type 1B",
  "term_label": "signal transduction",
  "gene": "UniProtKB:Q6P2M8",
  "gene_symbol": "PNCK"
}